{
  "gene_name": "Neuroblastoma breakpoint family member 9",
  "gene": "UniProtKB:P0DPF3",
  "term_id": "UNKNOWN:0003",
  "gene_symbol": "NBPF9",
  "term_label": "Unknown cellular component"
}